{
  "gene_symbol": "ZNF431",
  "gene_name": "Zinc finger protein 431",
  "gene": "UniProtKB:Q8TF32",
  "term_id": "GO:0000981",
  "term_label": "DNA-binding transcription factor activity, RNA polymerase II-specific"
}